{
  "gene_name": "Cell division cycle protein 20 homolog B",
  "gene_symbol": "CDC20B",
  "term_id": "GO:0005680",
  "term_label": "anaphase-promoting complex",
  "gene": "UniProtKB:Q86Y33"
}